{
  "gene_symbol": "SH2D7",
  "term_label": "protein-macromolecule adaptor activity",
  "gene": "UniProtKB:A6NKC9",
  "term_id": "GO:0030674",
  "gene_name": "SH2 domain-containing protein 7"
}